{
  "gene_symbol": "PF4V1",
  "term_label": "chemokine activity",
  "gene": "UniProtKB:P10720",
  "gene_name": "Platelet factor 4 variant",
  "term_id": "GO:0008009"
}